serine-phosphoethanolamine synthase activity [GO:0047494] (molecular function) Relationships: is_a phosphotransferase activity, for other substituted phosphate groups [GO:0016780] Also known as: CDP-ethanolamine:L-serine ethanolamine phosphotransferase activity, serine ethanolamine phosphate synthetase activity, serine ethanolamine phosphodiester synthase activity, serine ethanolaminephosphotransferase activity, serine-phosphinico-ethanolamine synthase activity, serinephosphoethanolamine synthase activity Sources: EC:2.7.8.4, RHEA:22656 Definition: Catalysis of the reaction: L-serine + CDP-ethanolamine = L-serine-phosphoethanolamine + CMP + H+.